{
  "gene_symbol": "MEOX2",
  "gene": "UniProtKB:P50222",
  "term_id": "GO:0000981",
  "term_label": "DNA-binding transcription factor activity, RNA polymerase II-specific",
  "gene_name": "Homeobox protein MOX-2"
}